{
  "gene_symbol": "CLP1",
  "term_id": "GO:0051731",
  "term_label": "polynucleotide 5'-hydroxyl-kinase activity",
  "gene_name": "Polyribonucleotide 5'-hydroxyl-kinase Clp1",
  "gene": "UniProtKB:Q92989"
}